{
  "term_id": "GO:0005886",
  "term_label": "plasma membrane",
  "gene": "UniProtKB:O00219",
  "gene_symbol": "HAS3",
  "gene_name": "Hyaluronan synthase 3"
}